{
  "gene_symbol": "ANXA2",
  "gene_name": "Annexin A2",
  "term_id": "GO:0005737",
  "gene": "UniProtKB:P07355",
  "term_label": "cytoplasm"
}